{
  "gene": "UniProtKB:Q6ZMT4",
  "gene_symbol": "KDM7A",
  "term_label": "Unknown cellular component",
  "term_id": "UNKNOWN:0003",
  "gene_name": "Lysine-specific demethylase 7A"
}